metanephric glomerular mesangial cell fate commitment [GO:0072256] (biological process) Relationships: is a type of glomerular mesangial cell fate commitment [GO:0072152]; is part of metanephric glomerular mesangial cell differentiation [GO:0072254] Sources: GOC:mtg_kidney_jan10 Definition: The process in which the developmental fate of a cell becomes restricted such that it will develop into a metanephric glomerular mesangial cell.